{
  "gene": "UniProtKB:O75600",
  "term_id": "GO:0005739",
  "gene_name": "2-amino-3-ketobutyrate coenzyme A ligase, mitochondrial",
  "gene_symbol": "GCAT",
  "term_label": "mitochondrion"
}